{
  "gene_name": "Serine protease inhibitor Kazal-type 1",
  "gene_symbol": "SPINK1",
  "term_id": "UNKNOWN:0001",
  "gene": "UniProtKB:P00995",
  "term_label": "Unknown molecular function"
}